cellular response to iron ion starvation [GO:0010106] (biological process) Regulation: regulated by regulation of cellular response to iron ion starvation [GO:1901966]; negatively regulated by negative regulation of cellular response to iron ion starvation [GO:1901967] Sources: GOC:mg Relationships: is a type of cellular response to starvation [GO:0009267]; is part of intracellular iron ion homeostasis [GO:0006879] Definition: Any process that results in a change in state or activity of a cell (in terms of movement, secretion, enzyme production, gene expression, etc.) as a result of deprivation of iron ions.